{
  "term_label": "postsynapse",
  "gene_name": "Striatin-4",
  "term_id": "GO:0098794",
  "gene_symbol": "STRN4",
  "gene": "UniProtKB:Q9NRL3"
}